{
  "gene_name": "Disks large-associated protein 1",
  "term_id": "GO:0050804",
  "term_label": "modulation of chemical synaptic transmission",
  "gene": "UniProtKB:O14490",
  "gene_symbol": "DLGAP1"
}